{
  "gene_symbol": "HARS2",
  "gene": "UniProtKB:P49590",
  "term_id": "GO:0005739",
  "term_label": "mitochondrion",
  "gene_name": "Histidine--tRNA ligase, mitochondrial"
}